negative regulation of eukaryotic translation initiation factor 4F complex assembly [GO:1905536] (biological process) Definition: Any process that stops, prevents or reduces the frequency, rate or extent of eukaryotic translation initiation factor 4F complex assembly. Relationships: is a type of GO:0031333; is a type of regulation of eukaryotic translation initiation factor 4F complex assembly [GO:1905535]; negatively regulates eukaryotic translation initiation factor 4F complex assembly [GO:0097010] Also known as: down regulation of eIF-4F assembly, down regulation of eIF4F assembly, down regulation of eukaryotic translation initiation factor 4F complex assembly, down-regulation of eIF-4F assembly, down-regulation of eIF4F assembly, down-regulation of eukaryotic translation initiation factor 4F complex assembly, downregulation of eIF-4F assembly, downregulation of eIF4F assembly, downregulation of eukaryotic translation initiation factor 4F complex assembly, negative regulation of eIF-4F assembly, negative regulation of eIF4F assembly, inhibition of eIF-4F assembly, inhibition of eIF4F assembly, inhibition of eukaryotic translation initiation factor 4F complex assembly References: PMID:18426977 Sources: GOC:PARL, GOC:TermGenie, GOC:bc, GO_REF:0000058